{
  "gene": "UniProtKB:Q70Z53",
  "term_label": "Unknown biological process",
  "gene_symbol": "FRA10AC1",
  "term_id": "UNKNOWN:0002",
  "gene_name": "Protein FRA10AC1"
}